{
  "gene_symbol": "ENTHD1",
  "term_id": "GO:0005886",
  "gene": "UniProtKB:Q8IYW4",
  "gene_name": "ENTH domain-containing protein 1",
  "term_label": "plasma membrane"
}